{
  "gene": "UniProtKB:Q2T9L4",
  "term_label": "postsynaptic density",
  "gene_symbol": "INSYN1",
  "gene_name": "Inhibitory synaptic factor 1",
  "term_id": "GO:0014069"
}